{
  "gene_symbol": "KMT5C",
  "gene": "UniProtKB:Q86Y97",
  "term_id": "GO:0005634",
  "gene_name": "Histone-lysine N-methyltransferase KMT5C",
  "term_label": "nucleus"
}